{
  "gene": "UniProtKB:P06748",
  "term_id": "GO:0045944",
  "term_label": "positive regulation of transcription by RNA polymerase II",
  "gene_symbol": "NPM1",
  "gene_name": "Nucleophosmin"
}